physiological cardiac muscle hypertrophy [GO:0003301] (biological process) Sources: GOC:BHF, GOC:mtg_cardiac_conduct_nov11, GOC:mtg_heart Relationships: is a type of GO:0003298; is a type of cardiac muscle hypertrophy [GO:0003300]; BFO_0000050 cardiac muscle tissue growth [GO:0055017] Definition: The enlargement or overgrowth of all or part of the heart muscle due to an increase in size of cardiac muscle cells without cell division. This process contributes to the developmental growth of the heart.